{
  "gene_name": "GAS2-like protein 2",
  "term_label": "stress fiber",
  "gene": "UniProtKB:Q8NHY3",
  "term_id": "GO:0001725",
  "gene_symbol": "GAS2L2"
}